histone H3K23ub reader activity [GO:0140257] (molecular function) Definition: A histone reader that recognizes a histone H3 ubiquitinated at lysine 23. References: PMID:29053958 Also known as: H3K23ub modified histone binding Note: Comment: Note that the residue position corresponds to the canonical human H3 histone (UniProtKB:P84243); this residue is conserved across all eukaryotes. Residue 1 is the first residue following removal of the initiating Methionine (Met). Note that each histone is encoded by multiple genes, and sequences may vary across different genes within an organism. Relationships: is a type of histone H3 reader activity [GO:0140006]